{
  "gene_symbol": "ODAPH",
  "term_id": "UNKNOWN:0003",
  "term_label": "Unknown cellular component",
  "gene_name": "Odontogenesis associated phosphoprotein",
  "gene": "UniProtKB:Q17RF5"
}